{
  "term_label": "Unknown biological process",
  "term_id": "UNKNOWN:0002",
  "gene_name": "Protein jagged-2",
  "gene_symbol": "JAG2",
  "gene": "UniProtKB:Q9Y219"
}